{
  "gene_name": "DnaJ homolog subfamily B member 4",
  "term_id": "GO:0051082",
  "gene": "UniProtKB:Q9UDY4",
  "gene_symbol": "DNAJB4",
  "term_label": "unfolded protein binding"
}